protein C inhibitor-PLAU complex [GO:0036027] (cellular component) References: PMID:10340997, PMID:3501295, PMID:8536714 Sources: GOC:ans Relationships: is a type of serine protease inhibitor complex [GO:0097180] Definition: A heterodimeric protein complex that contains protein C inhibitor (SERPINA5) and urokinase-type plasminogen activator (PLAU); formation of the complex inhibits the serine protease activity of urokinase-type plasminogen activator. Also known as: PCI-PLAU complex, SERPINA5-PLAU complex, plasma serine protease inhibitor-PLAU complex, protein C inhibitor-U-plasminogen activator complex, protein C inhibitor-uPA complex, protein C inhibitor-urokinase-type plasminogen activator complex, serpin A5-PLAU complex